{
  "term_label": "regulation of canonical Wnt signaling pathway",
  "gene": "UniProtKB:P0C7X3",
  "term_id": "GO:0060828",
  "gene_name": "Putative cyclin-Y-like protein 3",
  "gene_symbol": "CCNYL3"
}